{
  "term_label": "cytoplasm",
  "gene": "UniProtKB:H0Y7S4",
  "gene_name": "Putative PRAME family member 26",
  "gene_symbol": "PRAMEF26",
  "term_id": "GO:0005737"
}